{
  "gene": "UniProtKB:P13945",
  "gene_name": "Beta-3 adrenergic receptor",
  "term_id": "GO:0071880",
  "term_label": "adenylate cyclase-activating adrenergic receptor signaling pathway",
  "gene_symbol": "ADRB3"
}